dATP binding [GO:0032564] (molecular function) Sources: GOC:mah Relationships: is a type of adenyl deoxyribonucleotide binding [GO:0032558]; is a type of anion binding [GO:0043168] Definition: Binding to dATP, deoxyadenosine triphosphate.